{
  "gene": "UniProtKB:Q99689",
  "term_id": "UNKNOWN:0002",
  "gene_symbol": "FEZ1",
  "gene_name": "Fasciculation and elongation protein zeta-1",
  "term_label": "Unknown biological process"
}